{
  "gene_name": "Protocadherin beta-8",
  "gene_symbol": "PCDHB8",
  "gene": "UniProtKB:Q9UN66",
  "term_id": "GO:0050839",
  "term_label": "cell adhesion molecule binding"
}